{
  "term_id": "UNKNOWN:0001",
  "term_label": "Unknown molecular function",
  "gene": "UniProtKB:Q8N4V1",
  "gene_symbol": "MMGT1",
  "gene_name": "ER membrane protein complex subunit 5"
}